ovarian cumulus expansion [GO:0001550] (biological process) Relationships: is a type of ovulation cycle process [GO:0022602]; is_a developmental growth [GO:0048589]; is part of antral ovarian follicle growth [GO:0001547]; is part of fused antrum stage [GO:0048165] Definition: Increase in size of the cumulus surrounding the oocyte including change in morphology due to proliferation and dispersion of cumulus cells. Also known as: ovarian cumulus growth References: PMID:30010832